{
  "gene": "UniProtKB:P48448",
  "gene_name": "Aldehyde dehydrogenase family 3 member B2",
  "gene_symbol": "ALDH3B2",
  "term_id": "GO:0004029",
  "term_label": "aldehyde dehydrogenase (NAD+) activity"
}